{
  "gene_name": "Protein HRURF",
  "term_id": "UNKNOWN:0003",
  "gene_symbol": "HRURF",
  "term_label": "Unknown cellular component",
  "gene": "UniProtKB:P0DUH7"
}